{
  "term_id": "GO:0006355",
  "gene_name": "GON-4-like protein",
  "term_label": "regulation of DNA-templated transcription",
  "gene": "UniProtKB:Q3T8J9",
  "gene_symbol": "GON4L"
}